{
  "gene": "UniProtKB:O15342",
  "gene_name": "V-type proton ATPase subunit e 1",
  "term_label": "proton transmembrane transport",
  "term_id": "GO:1902600",
  "gene_symbol": "ATP6V0E1"
}